{
  "gene_name": "Proline and serine-rich protein 1",
  "gene_symbol": "PROSER1",
  "term_id": "UNKNOWN:0003",
  "term_label": "Unknown cellular component",
  "gene": "UniProtKB:Q86XN7"
}